{
  "term_label": "Unknown molecular function",
  "gene_symbol": "TAF1A",
  "gene_name": "TATA box-binding protein-associated factor RNA polymerase I subunit A",
  "gene": "UniProtKB:Q15573",
  "term_id": "UNKNOWN:0001"
}